{
  "gene_name": "Cytochrome c oxidase subunit 7C, mitochondrial",
  "term_id": "GO:0006123",
  "gene_symbol": "COX7C",
  "term_label": "mitochondrial electron transport, cytochrome c to oxygen",
  "gene": "UniProtKB:P15954"
}